{
  "gene_symbol": "ASCL2",
  "gene_name": "Achaete-scute homolog 2",
  "term_id": "GO:0000977",
  "gene": "UniProtKB:Q99929",
  "term_label": "RNA polymerase II transcription regulatory region sequence-specific DNA binding"
}